{
  "gene_symbol": "SV2C",
  "term_label": "regulation of synaptic vesicle exocytosis",
  "term_id": "GO:2000300",
  "gene_name": "Synaptic vesicle glycoprotein 2C",
  "gene": "UniProtKB:Q496J9"
}